{
  "gene_name": "Bromodomain adjacent to zinc finger domain protein 2A",
  "gene_symbol": "BAZ2A",
  "term_label": "rDNA heterochromatin",
  "term_id": "GO:0033553",
  "gene": "UniProtKB:Q9UIF9"
}